{
  "term_label": "histone binding",
  "gene_name": "Deubiquitinase MYSM1",
  "gene": "UniProtKB:Q5VVJ2",
  "gene_symbol": "MYSM1",
  "term_id": "GO:0042393"
}